bis-gamma-L-glutamylcystine reductase (NADPH) activity [GO:0047135] (molecular function) Definition: Catalysis of the reaction: 2 L-gamma-glutamyl-L-cysteine + NADP+ = bis-gamma-glutamylcystine + H+ + NADPH. Sources: EC:1.8.1.13, RHEA:11980 Relationships: is a type of oxidoreductase activity, acting on a sulfur group of donors, NAD(P) as acceptor [GO:0016668] Also known as: bis-g-glutamylcystine reductase (NADPH) activity, Bis-gamma-glutamylcystine reductase (NADPH), NADPH2:bis-gamma-glutamylcysteine oxidoreductase activity, NADPH:bis-gamma-glutamylcysteine oxidoreductase activity, bis-gamma-glutamylcystine reductase (NADPH) activity, gamma-glutamylcysteine:NADP+ oxidoreductase activity